negative regulation of CD4-positive, CD25-positive, alpha-beta regulatory T cell differentiation involved in immune response [GO:0032833] (biological process) Sources: GOC:mah Relationships: is a type of GO:0002698; is a type of negative regulation of CD4-positive, CD25-positive, alpha-beta regulatory T cell differentiation [GO:0032830]; is_a GO:0032832; is a type of negative regulation of immune response [GO:0050777]; negatively regulates GO:0002298 Also known as: inhibition of CD4-positive, CD25-positive, alpha-beta regulatory T cell differentiation during immune response, down regulation of CD4-positive, CD25-positive, alpha-beta regulatory T cell differentiation during immune response, down-regulation of CD4-positive, CD25-positive, alpha-beta regulatory T cell differentiation during immune response, downregulation of CD4-positive, CD25-positive, alpha-beta regulatory T cell differentiation during immune response, negative regulation of CD4-positive, CD25-positive, alpha-beta regulatory T cell development involved in immune response, negative regulation of CD4-positive, CD25-positive, alpha-beta regulatory T cell differentiation during immune response, negative regulation of CD4-positive, CD25-positive, alpha-beta regulatory T lymphocyte differentiation during immune response, negative regulation of CD4-positive, CD25-positive, alpha-beta regulatory T-cell differentiation during immune response, negative regulation of CD4-positive, CD25-positive, alpha-beta regulatory T-lymphocyte differentiation during immune response Definition: Any process that stops, prevents, or reduces the frequency, rate or extent of differentiation of CD4-positive, CD25-positive, alpha-beta regulatory T cells as part of an immune response. Note: Note that immunologists typically use the word 'development' to refer to cells of B or T cell lineages undergoing the process that GO describes as 'cell differentiation'.